{
  "gene_symbol": "BECN2",
  "term_label": "late endosome to vacuole transport",
  "gene": "UniProtKB:A8MW95",
  "gene_name": "Beclin-2",
  "term_id": "GO:0045324"
}